{
  "gene_name": "Arylsulfatase A",
  "term_id": "UNKNOWN:0002",
  "term_label": "Unknown biological process",
  "gene": "UniProtKB:P15289",
  "gene_symbol": "ARSA"
}